{
  "term_label": "Unknown molecular function",
  "gene_name": "Leukemia-associated protein 1",
  "gene": "UniProtKB:O43261",
  "term_id": "UNKNOWN:0001",
  "gene_symbol": "DLEU1"
}